high-affinity phosphate transmembrane transporter activity [GO:0048249] (molecular function) Relationships: is a type of phosphate transmembrane transporter activity [GO:0005315] Also known as: high affinity phosphate transmembrane transporter activity Definition: Enables the transfer of phosphate from one side of a membrane to the other. In high-affinity transport the transporter is able to bind the solute even if it is only present at very low concentrations. References: PMID:8709965 Sources: GOC:jid